alpha-beta T cell proliferation [GO:0046633] (biological process) Subtypes: NK T cell proliferation [GO:0001866], GO:0002310, CD4-positive, alpha-beta T cell proliferation [GO:0035739], CD8-positive, alpha-beta T cell proliferation [GO:0035740] Relationships: is_a T cell proliferation [GO:0042098]; is a type of alpha-beta T cell activation [GO:0046631] Also known as: alpha-beta T lymphocyte proliferation, alpha-beta T-cell proliferation, alpha-beta T-lymphocyte proliferation Sources: GOC:ai Definition: The expansion of an alpha-beta T cell population by cell division. Regulation: regulated by regulation of alpha-beta T cell proliferation [GO:0046640]; RO_0002213 by positive regulation of alpha-beta T cell proliferation [GO:0046641]; negatively regulated by GO:0046642